{
  "gene": "UniProtKB:Q6ZP68",
  "gene_symbol": "ATP11AUN",
  "gene_name": "Putative protein ATP11AUN",
  "term_label": "Unknown cellular component",
  "term_id": "UNKNOWN:0003"
}